{
  "gene_symbol": "WIZ",
  "gene": "UniProtKB:O95785",
  "term_label": "regulation of transcription by RNA polymerase II",
  "term_id": "GO:0006357",
  "gene_name": "Protein Wiz"
}